glutamate-cysteine ligase regulator activity [GO:1990609] (molecular function) References: PMID:8103521 Relationships: is a type of ligase regulator activity [GO:0055103]; RO_0002211 GO:0004357 Definition: Binds to and modulates the activity of glutamate-cysteine ligase.